{
  "gene_name": "Transcription factor Spi-B",
  "gene": "UniProtKB:Q01892",
  "term_id": "GO:0005634",
  "gene_symbol": "SPIB",
  "term_label": "nucleus"
}